{
  "gene_name": "Coiled-coil domain-containing protein 69",
  "term_id": "GO:0005737",
  "gene": "UniProtKB:A6NI79",
  "term_label": "cytoplasm",
  "gene_symbol": "CCDC69"
}